{
  "gene": "UniProtKB:P38646",
  "term_label": "ATP hydrolysis activity",
  "gene_name": "Stress-70 protein, mitochondrial",
  "term_id": "GO:0016887",
  "gene_symbol": "HSPA9"
}